delta-catenin binding [GO:0070097] (molecular function) Definition: Binding to the delta subunit of the catenin complex. Sources: GOC:rph Relationships: is a type of protein binding [GO:0005515]